{
  "gene_symbol": "CDH4",
  "gene": "UniProtKB:P55283",
  "gene_name": "Cadherin-4",
  "term_label": "cadherin binding",
  "term_id": "GO:0045296"
}